{
  "term_id": "GO:0000978",
  "term_label": "RNA polymerase II cis-regulatory region sequence-specific DNA binding",
  "gene_name": "Transcription factor NF-E2 45 kDa subunit",
  "gene_symbol": "NFE2",
  "gene": "UniProtKB:Q16621"
}